{
  "gene": "UniProtKB:P53007",
  "gene_symbol": "SLC25A1",
  "term_label": "mitochondrion",
  "gene_name": "Tricarboxylate transport protein, mitochondrial",
  "term_id": "GO:0005739"
}